3-hydroxybenzyl-alcohol dehydrogenase activity [GO:0047048] (molecular function) Relationships: is a type of oxidoreductase activity, acting on the CH-OH group of donors, NAD or NADP as acceptor [GO:0016616] Also known as: 3-hydroxybenzyl-alcohol:NADP+ oxidoreductase activity, m-hydroxybenzyl alcohol (NADP) dehydrogenase activity, m-hydroxybenzyl alcohol dehydrogenase activity, m-hydroxybenzylalcohol dehydrogenase activity Definition: Catalysis of the reaction: 3-hydroxybenzyl alcohol + NADP+ = 3-hydroxybenzaldehyde + H+ + NADPH. Sources: EC:1.1.1.97, RHEA:22340